regulation of hepatocyte growth factor receptor signaling pathway [GO:1902202] (biological process) Also known as: regulation of HGF receptor signaling pathway, regulation of HGF receptor signalling pathway, regulation of Met signaling pathway Definition: Any process that modulates the frequency, rate or extent of hepatocyte growth factor receptor signaling pathway. Subtypes: negative regulation of hepatocyte growth factor receptor signaling pathway [GO:1902203], positive regulation of hepatocyte growth factor receptor signaling pathway [GO:1902204] References: PMID:18819921 Sources: GOC:TermGenie Relationships: is a type of regulation of signal transduction [GO:0009966]; regulates hepatocyte growth factor receptor signaling pathway [GO:0048012]